endocardial precursor cell differentiation [GO:0003255] (biological process) Definition: The process in which a relatively unspecialized mesodermal cell acquires the specialized structural and/or functional features of an endocardial precursor cell. A endocardial precursor cell is a cell that has been committed to a endocardial cell fate, but will undergo further cell divisions rather than terminally differentiate. Relationships: is a type of cardioblast differentiation [GO:0010002] Sources: GOC:mtg_heart